{
  "gene": "UniProtKB:P20472",
  "gene_name": "Parvalbumin alpha",
  "gene_symbol": "PVALB",
  "term_id": "GO:0005509",
  "term_label": "calcium ion binding"
}